{
  "gene": "UniProtKB:O43435",
  "term_label": "nucleus",
  "gene_name": "T-box transcription factor TBX1",
  "gene_symbol": "TBX1",
  "term_id": "GO:0005634"
}